plasma membrane selenite transport [GO:0097080] (BP) Definition: The directed movement of inorganic selenite (HSeO3-1 at physiological pH) across a plasma membrane. Also known as: plasma membrane hydrogenselenite transport Relationships: is a type of transmembrane transport [GO:0055085] References: PMID:20861301 Sources: GOC:mcc